{
  "gene_symbol": "METAP2",
  "term_label": "aminopeptidase activity",
  "gene_name": "Methionine aminopeptidase 2",
  "term_id": "GO:0004177",
  "gene": "UniProtKB:P50579"
}